{
  "gene": "UniProtKB:Q5FWE3",
  "term_label": "Unknown molecular function",
  "gene_name": "Proline-rich transmembrane protein 3",
  "term_id": "UNKNOWN:0001",
  "gene_symbol": "PRRT3"
}